{
  "term_label": "calcium ion binding",
  "gene": "UniProtKB:Q9BUA6",
  "term_id": "GO:0005509",
  "gene_name": "Myosin regulatory light chain 10",
  "gene_symbol": "MYL10"
}